{
  "gene_symbol": "SYNCRIP",
  "gene": "UniProtKB:O60506",
  "gene_name": "Heterogeneous nuclear ribonucleoprotein Q",
  "term_label": "CRD-mediated mRNA stability complex",
  "term_id": "GO:0070937"
}